{
  "term_id": "GO:0002430",
  "gene_name": "Probable G-protein coupled receptor 33",
  "term_label": "complement receptor mediated signaling pathway",
  "gene": "UniProtKB:Q49SQ1",
  "gene_symbol": "GPR33"
}